{
  "gene_name": "Transcription factor AP-2-beta",
  "gene": "UniProtKB:Q92481",
  "gene_symbol": "TFAP2B",
  "term_label": "positive regulation of transcription by RNA polymerase II",
  "term_id": "GO:0045944"
}